{
  "gene_symbol": "ZNF785",
  "term_label": "regulation of transcription by RNA polymerase II",
  "gene_name": "Zinc finger protein 785",
  "gene": "UniProtKB:A8K8V0",
  "term_id": "GO:0006357"
}